{
  "term_label": "nuclear speck",
  "gene_name": "Splicing factor U2AF 65 kDa subunit",
  "gene_symbol": "U2AF2",
  "gene": "UniProtKB:P26368",
  "term_id": "GO:0016607"
}